organelle [GO:0043226] (cellular component) Relationships: is a type of GO:0110165 Definition: Organized structure of distinctive morphology and function. Includes the nucleus, mitochondria, plastids, vacuoles, vesicles, ribosomes and the cytoskeleton, and prokaryotic structures such as anammoxosomes and pirellulosomes. Excludes the plasma membrane. Sources: GOC:go_curators Subtypes: GO:0043227, membraneless organelle [GO:0043228], intracellular organelle [GO:0043229], extracellular organelle [GO:0043230], postsynaptic specialization [GO:0099572]